heparan sulfate N-deacetylase activity [GO:0102140] (molecular function) Sources: RHEA:70587 Definition: Catalysis of the reaction: H2O + [heparan sulfate]-N-acetyl-alpha-D-glucosamine = acetate + H+ + [heparan sulfate]-alpha-D-glucosamine. Relationships: is a type of deacetylase activity [GO:0019213]; is a type of carboxylic ester hydrolase activity [GO:0052689]